{
  "term_label": "ATP binding",
  "gene": "UniProtKB:P07900",
  "gene_symbol": "HSP90AA1",
  "term_id": "GO:0005524",
  "gene_name": "Heat shock protein HSP 90-alpha"
}